{
  "term_label": "Unknown cellular component",
  "gene": "UniProtKB:A6NHN6",
  "gene_name": "Nuclear pore complex-interacting protein family member B15",
  "term_id": "UNKNOWN:0003",
  "gene_symbol": "NPIPB15"
}